UDP-glucose transmembrane transport into endoplasmic reticulum [GO:0120112] (biological process) Definition: The directed movement of UDP-glucose from cytosol to endoplasmic reticulum. Relationships: is a type of UDP-glucose transmembrane transport [GO:0015786]; is a type of GO:0046967 References: PMID:27587357